{
  "term_label": "Unknown cellular component",
  "gene_name": "CPX chromosomal region candidate gene 1 protein",
  "gene": "UniProtKB:Q8N123",
  "gene_symbol": "CPXCR1",
  "term_id": "UNKNOWN:0003"
}